{
  "gene_symbol": "DNAH3",
  "gene": "UniProtKB:Q8TD57",
  "gene_name": "Dynein axonemal heavy chain 3",
  "term_label": "dynein light intermediate chain binding",
  "term_id": "GO:0051959"
}